{
  "gene_symbol": "CFAP144",
  "term_label": "Unknown molecular function",
  "term_id": "UNKNOWN:0001",
  "gene": "UniProtKB:A6NL82",
  "gene_name": "Cilia- and flagella-associated protein 144"
}